{
  "term_id": "GO:2001204",
  "gene_symbol": "SIGLEC15",
  "gene": "UniProtKB:Q6ZMC9",
  "term_label": "regulation of osteoclast development",
  "gene_name": "Sialic acid-binding Ig-like lectin 15"
}